{
  "term_id": "UNKNOWN:0003",
  "gene_name": "Vesicle transport protein SFT2B",
  "gene": "UniProtKB:O95562",
  "gene_symbol": "SFT2D2",
  "term_label": "Unknown cellular component"
}